{
  "term_id": "UNKNOWN:0001",
  "term_label": "Unknown molecular function",
  "gene": "UniProtKB:Q5VXM1",
  "gene_name": "CUB domain-containing protein 2",
  "gene_symbol": "CDCP2"
}